1,2-beta-fructan 1F-fructosyltransferase activity [GO:0047207] (molecular function) Also known as: 1,2-beta-D-fructan 1(F)-fructosyltransferase activity, 1,2-beta-D-fructan 1F-fructosyltransferase activity, 1,2-beta-D-fructan:1,2-beta-D-fructan 1(F)-beta-D-fructosyltransferase activity, 1,2-beta-D-fructan:1,2-beta-D-fructan 1F-beta-D-fructosyltransferase activity, 1,2-beta-fructan 1(F)-fructosyltransferase activity, 2,1-beta-D-fructan:2,1-beta-D-fructan 1-beta-D-fructosyltransferase activity, 2,1-fructan:2,1-fructan 1-fructosyltransferase activity, FFT activity, fructan:fructan fructosyl transferase activity Definition: Catalysis of the reaction: [(1->2)-beta-D-fructosyl](n) + [(1->2)-beta-D-fructosyl](m) = [(1->2)-beta-D-fructosyl](n+1) + [(1->2)-beta-D-fructosyl](m-1). Sources: EC:2.4.1.100, MetaCyc:2.4.1.100-RXN Relationships: is a type of fructosyltransferase activity [GO:0050738]